mitochondrial mRNA 5'-end processing [GO:0090617] (biological process) Definition: Any process involved in forming the mature 5' end of an mRNA molecule that derives from the mitochondrial genome. References: PMID:25181358 Sources: GOC:tb Relationships: is a type of GO:0090615